{
  "gene_symbol": "ZAR1",
  "term_id": "GO:0005737",
  "gene": "UniProtKB:Q86SH2",
  "gene_name": "Zygote arrest protein 1",
  "term_label": "cytoplasm"
}